extrahaustorial matrix [GO:0085036] (cellular component) Note: See also: haustorium ; GO:0085035 and extrahaustorial membrane ; GO:0085037. Definition: The space between the symbiont plasma membrane and the extrahaustorial membrane of the host. Sources: GOC:pamgo_curators Relationships: is a type of cellular anatomical structure [GO:0110165]; is part of extracellular region [GO:0005576]; BFO_0000050 host extracellular space [GO:0043655]